{
  "gene_name": "CD2-associated protein",
  "term_id": "GO:0005886",
  "gene_symbol": "CD2AP",
  "term_label": "plasma membrane",
  "gene": "UniProtKB:Q9Y5K6"
}